axon midline choice point recognition [GO:0016199] (biological process) Relationships: is a type of axon choice point recognition [GO:0016198] Definition: The recognition of molecules at the central nervous system midline choice point by an axon growth cone; this choice point determines whether the growth cone will cross the midline. References: PMID:11376484 Subtypes: corticospinal neuron axon decussation [GO:0021973]